{
  "gene": "UniProtKB:Q92953",
  "term_id": "GO:0043025",
  "gene_symbol": "KCNB2",
  "term_label": "neuronal cell body",
  "gene_name": "Potassium voltage-gated channel subfamily B member 2"
}